{
  "gene": "UniProtKB:P35716",
  "term_id": "GO:0048593",
  "term_label": "camera-type eye morphogenesis",
  "gene_name": "Transcription factor SOX-11",
  "gene_symbol": "SOX11"
}